{
  "term_label": "peptide hormone binding",
  "term_id": "GO:0017046",
  "gene_name": "Vasoactive intestinal polypeptide receptor 1",
  "gene": "UniProtKB:P32241",
  "gene_symbol": "VIPR1"
}